postsynaptic membrane [GO:0045211] (cellular component) Relationships: is a type of GO:0097060; is part of GO:0098794 Also known as: post-synaptic membrane Sources: ISBN:0198506732 Definition: A specialized area of membrane facing the presynaptic membrane on the tip of the nerve ending and separated from it by a minute cleft (the synaptic cleft). Neurotransmitters cross the synaptic cleft and transmit the signal to the postsynaptic membrane.